{
  "gene_symbol": "PITPNC1",
  "gene": "UniProtKB:Q9UKF7",
  "term_label": "cytoplasm",
  "gene_name": "Cytoplasmic phosphatidylinositol transfer protein 1",
  "term_id": "GO:0005737"
}